{
  "gene_symbol": "WDR55",
  "gene": "UniProtKB:Q9H6Y2",
  "term_id": "UNKNOWN:0002",
  "term_label": "Unknown biological process",
  "gene_name": "WD repeat-containing protein 55"
}